membrane-enclosed lumen [GO:0031974] (cellular component) Sources: GOC:add, GOC:mah Relationships: is a type of cellular anatomical structure [GO:0110165] Definition: The enclosed volume within a sealed membrane or between two sealed membranes. Encompasses the volume enclosed by the membranes of a particular organelle, e.g. endoplasmic reticulum lumen, or the space between the two lipid bilayers of a double membrane surrounding an organelle, e.g. nuclear envelope lumen. Subtypes: GO:0020004, organelle lumen [GO:0043233], pathogen-containing vacuole lumen [GO:0140222]